regulation of synaptic vesicle exocytosis [GO:2000300] (biological process) Definition: Any process that modulates the frequency, rate or extent of synaptic vesicle exocytosis. Relationships: is_a regulation of neurotransmitter secretion [GO:0046928]; is a type of regulation of regulated secretory pathway [GO:1903305]; regulates synaptic vesicle exocytosis [GO:0016079] Subtypes: regulation of calcium ion-dependent exocytosis of neurotransmitter [GO:1903233], GO:2000301, GO:2000302 Sources: GOC:obol